{
  "gene_name": "Caspase recruitment domain-containing protein 6",
  "term_id": "UNKNOWN:0001",
  "term_label": "Unknown molecular function",
  "gene_symbol": "CARD6",
  "gene": "UniProtKB:Q9BX69"
}